{
  "gene_symbol": "CDC123",
  "gene_name": "Cell division cycle protein 123 homolog",
  "term_id": "UNKNOWN:0002",
  "term_label": "Unknown biological process",
  "gene": "UniProtKB:O75794"
}